{
  "term_label": "intracellular protein transport",
  "term_id": "GO:0006886",
  "gene_symbol": "RAB18",
  "gene": "UniProtKB:Q9NP72",
  "gene_name": "Ras-related protein Rab-18"
}